glutamate-cysteine ligase catalytic subunit binding [GO:0035226] (molecular function) Definition: Binding to the catalytic subunit of glutamate-cysteine ligase. Relationships: is_a enzyme binding [GO:0019899] References: PMID:12954617